{
  "term_label": "chromatin binding",
  "gene_name": "Protein polybromo-1",
  "term_id": "GO:0003682",
  "gene_symbol": "PBRM1",
  "gene": "UniProtKB:Q86U86"
}